{
  "gene": "UniProtKB:P02458",
  "term_label": "collagen type II trimer",
  "gene_symbol": "COL2A1",
  "gene_name": "Collagen alpha-1(II) chain",
  "term_id": "GO:0005585"
}